regulation of peptidyl-serine phosphorylation [GO:0033135] (biological process) Sources: GOC:mah Subtypes: GO:0033137, positive regulation of peptidyl-serine phosphorylation [GO:0033138], regulation of peptidyl-serine phosphorylation of STAT protein [GO:0033139] Relationships: is a type of regulation of protein phosphorylation [GO:0001932]; regulates GO:0018105 Definition: Any process that modulates the frequency, rate or extent of the phosphorylation of peptidyl-serine.